{
  "term_id": "GO:0030154",
  "gene": "UniProtKB:Q9NQI0",
  "term_label": "cell differentiation",
  "gene_symbol": "DDX4",
  "gene_name": "Probable ATP-dependent RNA helicase DDX4"
}